{
  "gene_name": "Olfactory receptor 10T2",
  "gene": "UniProtKB:Q8NGX3",
  "gene_symbol": "OR10T2",
  "term_id": "GO:0050911",
  "term_label": "detection of chemical stimulus involved in sensory perception of smell"
}